{
  "gene": "UniProtKB:P38919",
  "gene_name": "Eukaryotic initiation factor 4A-III",
  "term_id": "GO:0003724",
  "term_label": "RNA helicase activity",
  "gene_symbol": "EIF4A3"
}